{
  "gene_name": "Probable phospholipid-transporting ATPase IIB",
  "term_id": "GO:0045332",
  "term_label": "phospholipid translocation",
  "gene_symbol": "ATP9B",
  "gene": "UniProtKB:O43861"
}